{
  "gene": "UniProtKB:Q99961",
  "gene_name": "Endophilin-A2",
  "term_id": "GO:0098978",
  "gene_symbol": "SH3GL1",
  "term_label": "glutamatergic synapse"
}